phytosphingosine metabolic process [GO:0006671] (biological process) Definition: The chemical reactions and pathways involving phytosphingosine, (2S,3S,4R)-2-aminooctadecane-1,3,4-triol, a constituent of many plant sphingolipids. Also known as: phytosphingosine metabolism Relationships: is a type of polyol metabolic process [GO:0019751]; is a type of sphingoid metabolic process [GO:0046519] Subtypes: phytosphingosine biosynthetic process [GO:0071602] Sources: ISBN:0198506732